{
  "gene_symbol": "SMCO2",
  "gene": "UniProtKB:A6NFE2",
  "term_id": "UNKNOWN:0002",
  "gene_name": "Single-pass membrane and coiled-coil domain-containing protein 2",
  "term_label": "Unknown biological process"
}